{
  "gene_symbol": "CCDC158",
  "gene_name": "Coiled-coil domain-containing protein 158",
  "term_label": "Unknown cellular component",
  "term_id": "UNKNOWN:0003",
  "gene": "UniProtKB:Q5M9N0"
}